{
  "gene_symbol": "MEF2C",
  "gene": "UniProtKB:Q06413",
  "gene_name": "Myocyte-specific enhancer factor 2C",
  "term_label": "cell differentiation",
  "term_id": "GO:0030154"
}